{
  "term_id": "UNKNOWN:0003",
  "gene": "UniProtKB:Q96JG9",
  "gene_symbol": "ZNF469",
  "gene_name": "Zinc finger protein 469",
  "term_label": "Unknown cellular component"
}